positive regulation of heart rate by norepinephrine [GO:0003066] (biological process) Subtypes: GO:0003113, positive regulation of heart rate by circulating norepinephrine [GO:0003114] Also known as: noradrenaline cardiac chronotropy, noradrenaline regulation of the rate of heart muscle contraction, norepinephrine cardiac chronotropy, positive regulation of heart rate by adrenaline, positive regulation of heart contraction rate by norepinephrine Definition: The process in which the secretion of norepinephrine into the bloodstream or released from nerve endings increases the rate of heart muscle contraction. Sources: GOC:mtg_cardio, GOC:rl Relationships: is a type of regulation of heart rate by chemical signal [GO:0003062]; is a type of positive regulation of heart rate [GO:0010460]; is part of GO:0001996